{
  "gene_name": "Stimulated by retinoic acid gene 8 protein homolog",
  "term_id": "GO:0007283",
  "term_label": "spermatogenesis",
  "gene_symbol": "STRA8",
  "gene": "UniProtKB:Q7Z7C7"
}